{
  "gene_symbol": "AZU1",
  "term_label": "protein maturation",
  "gene_name": "Azurocidin",
  "term_id": "GO:0051604",
  "gene": "UniProtKB:P20160"
}